{
  "term_id": "UNKNOWN:0001",
  "gene_name": "Interleukin-36 receptor antagonist protein",
  "gene_symbol": "IL36RN",
  "gene": "UniProtKB:Q9UBH0",
  "term_label": "Unknown molecular function"
}